{
  "gene": "UniProtKB:Q9ULW5",
  "gene_symbol": "RAB26",
  "gene_name": "Ras-related protein Rab-26",
  "term_label": "GTPase activity",
  "term_id": "GO:0003924"
}